{
  "term_label": "dynein intermediate chain binding",
  "term_id": "GO:0045505",
  "gene": "UniProtKB:Q96FJ2",
  "gene_name": "Dynein light chain 2, cytoplasmic",
  "gene_symbol": "DYNLL2"
}